{
  "gene_symbol": "FRMPD3",
  "gene_name": "FERM and PDZ domain-containing protein 3",
  "term_id": "UNKNOWN:0003",
  "gene": "UniProtKB:Q5JV73",
  "term_label": "Unknown cellular component"
}